regulation of deadenylation-dependent decapping of nuclear-transcribed mRNA [GO:0106288] (biological process) Subtypes: negative regulation of deadenylation-dependent decapping of nuclear-transcribed mRNA [GO:0106289] References: PMID:32354837 Definition: Any process that modulates the frequency, rate or extent of deadenylation-dependent decapping of nuclear-transcribed mRNA. Relationships: is a type of regulation of mRNA catabolic process [GO:0061013]; regulates deadenylation-dependent decapping of nuclear-transcribed mRNA [GO:0000290]